{
  "gene_name": "Retinol-binding protein 3",
  "gene": "UniProtKB:P10745",
  "term_label": "cone matrix sheath",
  "term_id": "GO:0090658",
  "gene_symbol": "RBP3"
}